{
  "term_label": "mitotic sister chromatid cohesion",
  "term_id": "GO:0007064",
  "gene_name": "N-acetyltransferase ESCO2",
  "gene": "UniProtKB:Q56NI9",
  "gene_symbol": "ESCO2"
}